{
  "gene": "UniProtKB:Q5JPI3",
  "term_label": "Unknown biological process",
  "gene_name": "Uncharacterized protein C3orf38",
  "gene_symbol": "C3orf38",
  "term_id": "UNKNOWN:0002"
}